{
  "gene_name": "TBC1 domain family member 12",
  "term_label": "recycling endosome",
  "gene": "UniProtKB:O60347",
  "term_id": "GO:0055037",
  "gene_symbol": "TBC1D12"
}